{
  "gene": "UniProtKB:P05023",
  "term_id": "GO:1902600",
  "term_label": "proton transmembrane transport",
  "gene_symbol": "ATP1A1",
  "gene_name": "Sodium_potassium-transporting ATPase subunit alpha-1"
}